{
  "gene_name": "NADH dehydrogenase [ubiquinone] 1 alpha subcomplex assembly factor 2",
  "gene_symbol": "NDUFAF2",
  "term_id": "GO:0005739",
  "term_label": "mitochondrion",
  "gene": "UniProtKB:Q8N183"
}